{
  "term_id": "GO:0005634",
  "term_label": "nucleus",
  "gene": "UniProtKB:Q8WVM7",
  "gene_symbol": "STAG1",
  "gene_name": "Cohesin subunit SA-1"
}